proton-transporting two-sector ATPase complex, proton-transporting domain [GO:0033177] (cellular component) Definition: A protein complex that forms part of a proton-transporting two-sector ATPase complex and carries out proton transport across a membrane. The proton-transporting domain (F0, V0, or A0) includes integral and peripheral membrane proteins. Subtypes: GO:0033179 References: PMID:10838056 Sources: GOC:mah Relationships: is_a membrane protein complex [GO:0098796]; is part of proton-transporting two-sector ATPase complex [GO:0016469]